methionyl glutamyl tRNA synthetase complex [GO:0017102] (cellular component) References: PMID:11069915 Sources: GOC:mcc Relationships: is a type of protein-containing complex [GO:0032991]; is part of cytoplasm [GO:0005737] Definition: A complex consisting of methionyl- and glutamyl-tRNA synthetases. The tRNA synthetases present in the complex bind to their cognate tRNAs more efficiently than they do as monomers.